{
  "gene_name": "Sodium-dependent phosphate transport protein 4",
  "term_label": "toxin transmembrane transporter activity",
  "gene_symbol": "SLC17A3",
  "term_id": "GO:0019534",
  "gene": "UniProtKB:O00476"
}